Holliday junction helicase complex [GO:0009379] (cellular component) References: PMID:16935884, PMID:9442895 Relationships: is a type of GO:0033202 Definition: A DNA helicase complex found at Holliday junctions where the helicase activity is involved in the migration of the junction branch point. The best-characterized example is the E. coli RuvAB complex, in which a hexamer of RuvB subunits possesses helicase activity that is modulated by association with RuvA.